{
  "gene_symbol": "PIGK",
  "gene_name": "GPI-anchor transamidase",
  "term_id": "GO:0003923",
  "gene": "UniProtKB:Q92643",
  "term_label": "GPI-anchor transamidase activity"
}